{
  "term_label": "Unknown cellular component",
  "gene": "UniProtKB:Q537H7",
  "gene_symbol": "SPATA45",
  "term_id": "UNKNOWN:0003",
  "gene_name": "Spermatogenesis-associated protein 45"
}